{
  "term_label": "Unknown molecular function",
  "gene": "UniProtKB:A0A075B6V8",
  "gene_symbol": "TRAJ5",
  "gene_name": "T cell receptor alpha joining 5 (Fragment)",
  "term_id": "UNKNOWN:0001"
}